{
  "gene_name": "Zinc finger and SCAN domain-containing protein 1",
  "gene_symbol": "ZSCAN1",
  "term_label": "regulation of transcription by RNA polymerase II",
  "term_id": "GO:0006357",
  "gene": "UniProtKB:Q8NBB4"
}